rod bipolar cell terminal bouton [GO:1990795] (cellular component) References: PMID:19883736 Relationships: is a type of GO:0043195 Definition: A specialized region of the axon terminus portion of a rod bipolar axon. A rod bipolar cell is a neuron found in the retina and having connections with rod photoreceptor cells and neurons in the inner plexiform layer.